positive regulation of blood vessel remodeling [GO:2000504] (biological process) Definition: Any process that activates or increases the frequency, rate or extent of blood vessel remodeling. Sources: GOC:obol Also known as: positive regulation of blood vessel remodelling Relationships: is a type of positive regulation of tissue remodeling [GO:0034105]; is_a GO:0060312; positively regulates blood vessel remodeling [GO:0001974] Subtypes: GO:1905111